{
  "term_id": "GO:0031122",
  "gene": "UniProtKB:Q8ND83",
  "gene_name": "SLAIN motif-containing protein 1",
  "term_label": "cytoplasmic microtubule organization",
  "gene_symbol": "SLAIN1"
}